negative regulation of chondrocyte hypertrophy [GO:1903042] (biological process) Relationships: is a type of negative regulation of cell growth [GO:0030308]; is_a negative regulation of developmental growth [GO:0048640]; is a type of negative regulation of chondrocyte development [GO:0061182]; is a type of GO:1903041; negatively regulates chondrocyte hypertrophy [GO:0003415] Also known as: down regulation of chondrocyte hypertrophy, down-regulation of chondrocyte hypertrophy, downregulation of chondrocyte hypertrophy, inhibition of chondrocyte hypertrophy References: PMID:23928032 Sources: GOC:TermGenie, GOC:mr, GO_REF:0000058 Definition: Any process that stops, prevents or reduces the frequency, rate or extent of chondrocyte hypertrophy.